{
  "term_label": "nucleus",
  "gene": "UniProtKB:Q96CT7",
  "term_id": "GO:0005634",
  "gene_symbol": "CCDC124",
  "gene_name": "Coiled-coil domain-containing protein 124"
}